neurotransmitter receptor localization to postsynaptic specialization membrane [GO:0099645] (biological process) Definition: A process in which a neurotransmitter is transported to, or maintained in, a location within the membrane adjacent to a postsynaptic specialization (e.g. postsynaptic density). Also known as: neurotransmitter receptor localisation in postsynaptic specialization membrane Relationships: is a type of protein-containing complex localization [GO:0031503]; is a type of receptor localization to synapse [GO:0097120]; is a type of regulation of postsynaptic membrane neurotransmitter receptor levels [GO:0099072]; is a type of GO:0099633 Sources: GOC:dos Regulation: regulated by regulation of neurotransmitter receptor localization to postsynaptic specialization membrane [GO:0098696]